{
  "term_label": "nucleus",
  "gene_symbol": "TEF",
  "gene_name": "Thyrotroph embryonic factor",
  "gene": "UniProtKB:Q10587",
  "term_id": "GO:0005634"
}